{
  "gene_symbol": "KRT15",
  "term_id": "GO:0002009",
  "gene": "UniProtKB:P19012",
  "term_label": "morphogenesis of an epithelium",
  "gene_name": "Keratin, type I cytoskeletal 15"
}